ureter urothelium development [GO:0072190] (biological process) Also known as: ureter epithelium development Definition: The process whose specific outcome is the progression of the urothelium of the ureter over time, from its formation to the mature structure. The urothelium is an epithelium that makes up the epithelial tube of the ureter. Relationships: is a type of epithelium development [GO:0060429]; is part of ureter development [GO:0072189] Sources: GOC:mtg_kidney_jan10